ribonucleoside-diphosphate reductase complex [GO:0005971] (cellular component) References: PMID:10716984, PMID:21336276 Relationships: is a type of oxidoreductase complex [GO:1990204]; is part of cytosol [GO:0005829] Also known as: RNR complex, ribonucleotide reductase complex Definition: An enzyme complex composed of 2-4 or more subunits, which usually contains nonheme iron and requires ATP for catalysis. Catalyzes the formation of 2'-deoxyribonucleoside diphosphate from ribonucleoside diphosphate, using either thioredoxin disulfide or glutaredoxin disulfide as an acceptor.